response to L-glutamate [GO:1902065] (biological process) Definition: Any process that results in a change in state or activity of a cell or an organism (in terms of movement, secretion, enzyme production, gene expression, etc.) as a result of an L-glutamate stimulus. Relationships: is a type of GO:0043200; is a type of response to nitrogen compound [GO:1901698]; is a type of response to oxygen-containing compound [GO:1901700] Subtypes: cellular response to L-glutamate [GO:1905232] References: PMID:23574009 Sources: GOC:TermGenie